consider [oboInOwl#consider]